{
  "gene": "UniProtKB:Q9NXB9",
  "term_label": "fatty acid elongation, polyunsaturated fatty acid",
  "gene_name": "Elongation of very long chain fatty acids protein 2",
  "gene_symbol": "ELOVL2",
  "term_id": "GO:0034626"
}